cytoskeletal protein-membrane anchor activity [GO:0106006] (molecular function) Definition: The binding activity of a molecule that brings together a cytoskeletal protein or protein complex and a plasma membrane lipid or membrane-associated protein, in order to maintain the localization of the cytoskeleton at a specific cortical membrane location. References: PMID:25736293, PMID:30840879 Also known as: cytoskeletal protein membrane adaptor, cytoskeletal protein membrane anchor activity, cytoskeletal protein membrane tether activity, cytoskeletal protein-membrane adaptor activity, membrane-cytoskeletal protein anchor activity, membrane-cytoskeletal protein tether activity, cytoskeletal protein to membrane recruiting activity, BAR domain adaptor, F-BAR domain adaptor, microtubule cortical anchor activity Relationships: is a type of cytoskeletal anchor activity [GO:0008093]; is a type of protein-membrane adaptor activity [GO:0043495]; has part GO:0008289